{
  "gene_symbol": "ADAM20",
  "term_id": "GO:0009897",
  "term_label": "external side of plasma membrane",
  "gene": "UniProtKB:O43506",
  "gene_name": "Disintegrin and metalloproteinase domain-containing protein 20"
}